{
  "term_id": "GO:0023026",
  "gene": "UniProtKB:P79483",
  "term_label": "MHC class II protein complex binding",
  "gene_symbol": "HLA-DRB3",
  "gene_name": "HLA class II histocompatibility antigen, DR beta 3 chain"
}